{
  "term_id": "GO:0005009",
  "gene": "UniProtKB:P08069",
  "term_label": "insulin receptor activity",
  "gene_symbol": "IGF1R",
  "gene_name": "Insulin-like growth factor 1 receptor"
}